{
  "gene": "UniProtKB:P23634",
  "term_id": "GO:0005388",
  "gene_symbol": "ATP2B4",
  "gene_name": "Plasma membrane calcium-transporting ATPase 4",
  "term_label": "P-type calcium transporter activity"
}